{
  "gene_symbol": "PAPPA",
  "gene": "UniProtKB:Q13219",
  "term_label": "cell surface receptor signaling pathway",
  "term_id": "GO:0007166",
  "gene_name": "Pappalysin-1"
}